{
  "gene_name": "Vesicular glutamate transporter 3",
  "term_id": "GO:0005326",
  "gene_symbol": "SLC17A8",
  "gene": "UniProtKB:Q8NDX2",
  "term_label": "neurotransmitter transmembrane transporter activity"
}